maintenance of protein location in cell cortex [GO:0032065] (biological process) Definition: A process in which a protein or protein complex is maintained in a specific location in the cell cortex. Subtypes: maintenance of protein location in cell cortex of cell tip [GO:0097248] Sources: GOC:vw Also known as: cortical protein anchoring Relationships: is a type of GO:0032507; occurs in GO:0005938